{
  "term_id": "UNKNOWN:0001",
  "term_label": "Unknown molecular function",
  "gene_name": "Keratinocyte differentiation factor 1",
  "gene_symbol": "KDF1",
  "gene": "UniProtKB:Q8NAX2"
}